{
  "term_id": "GO:0045429",
  "gene_symbol": "DDAH1",
  "gene": "UniProtKB:O94760",
  "term_label": "positive regulation of nitric oxide biosynthetic process",
  "gene_name": "N(G),N(G)-dimethylarginine dimethylaminohydrolase 1"
}